{
  "gene_name": "DNA topoisomerase 2-beta",
  "gene_symbol": "TOP2B",
  "gene": "UniProtKB:Q02880",
  "term_label": "sister chromatid segregation",
  "term_id": "GO:0000819"
}